{
  "gene_name": "Procollagen-lysine,2-oxoglutarate 5-dioxygenase 1",
  "gene": "UniProtKB:Q02809",
  "term_label": "collagen fibril organization",
  "term_id": "GO:0030199",
  "gene_symbol": "PLOD1"
}